{
  "gene_name": "DNA repair endonuclease XPF",
  "gene_symbol": "ERCC4",
  "term_label": "nucleotide-excision repair factor 1 complex",
  "gene": "UniProtKB:Q92889",
  "term_id": "GO:0000110"
}